germinal center formation [GO:0002467] (BP) Definition: The process in which germinal centers form. A germinal center is a specialized microenvironment formed when activated B cells enter lymphoid follicles. Germinal centers are the foci for B cell proliferation and somatic hypermutation. Relationships: is a type of adaptive immune response based on somatic recombination of immune receptors built from immunoglobulin superfamily domains [GO:0002460]; is_a anatomical structure formation involved in morphogenesis [GO:0048646] Sources: GOC:jal, GO_REF:0000022, ISBN:081533642X Regulation: regulated by regulation of germinal center formation [GO:0002634]; negatively regulated by negative regulation of germinal center formation [GO:0002635]; positively regulated by positive regulation of germinal center formation [GO:0002636]